{
  "gene_symbol": "C6orf132",
  "gene_name": "Uncharacterized protein C6orf132",
  "term_label": "Unknown molecular function",
  "term_id": "UNKNOWN:0001",
  "gene": "UniProtKB:Q5T0Z8"
}